common myeloid progenitor cell proliferation [GO:0035726] (BP) Definition: The multiplication or reproduction of common myeloid progenitor cells, resulting in the expansion of a cell population. A common myeloid progenitor cell is a progenitor cell committed to the myeloid lineage. Relationships: is a type of cell population proliferation [GO:0008283] Sources: CL:0000049, GOC:BHF